{
  "term_label": "Unknown cellular component",
  "gene": "UniProtKB:O95620",
  "gene_symbol": "DUS4L",
  "gene_name": "tRNA-dihydrouridine(20a_20b) synthase [NAD(P)+]-like",
  "term_id": "UNKNOWN:0003"
}